{
  "term_label": "cytoplasmic translation",
  "term_id": "GO:0002181",
  "gene_symbol": "DRG2",
  "gene": "UniProtKB:P55039",
  "gene_name": "Developmentally-regulated GTP-binding protein 2"
}